{
  "gene": "UniProtKB:P53041",
  "gene_name": "Serine_threonine-protein phosphatase 5",
  "gene_symbol": "PPP5C",
  "term_id": "GO:0004722",
  "term_label": "protein serine/threonine phosphatase activity"
}